purine ribonucleoside monophosphate catabolic process [GO:0009169] (biological process) Sources: GOC:go_curators, ISBN:0198506732 Definition: The chemical reactions and pathways resulting in the breakdown of purine ribonucleoside monophosphate, a compound consisting of a purine base linked to a ribose sugar esterified with phosphate on the sugar. Also known as: purine ribonucleoside monophosphate breakdown, purine ribonucleoside monophosphate catabolism, purine ribonucleoside monophosphate degradation Subtypes: GO:0006196, IMP catabolic process [GO:0006204], GMP catabolic process [GO:0046038] Relationships: is a type of purine nucleoside monophosphate catabolic process [GO:0009128]; is a type of ribonucleoside monophosphate catabolic process [GO:0009158]; is a type of purine ribonucleoside monophosphate metabolic process [GO:0009167]